guanosine pentaphosphate catabolic process [GO:0015974] (biological process) Sources: GOC:ai Definition: The chemical reactions and pathways resulting in the breakdown of guanine pentaphosphate (5'-pppGpp-3'), a derivative of guanine riboside with five phosphates. Relationships: is a type of purine ribonucleotide catabolic process [GO:0009154]; is a type of guanosine pentaphosphate metabolic process [GO:0015972]; is a type of purine ribonucleoside bisphosphate catabolic process [GO:0034037] Also known as: guanosine pentaphosphate (5'-pppGpp-3') catabolic process, guanosine pentaphosphate (5'-pppGpp-3') catabolism, guanosine pentaphosphate breakdown, guanosine pentaphosphate catabolism, guanosine pentaphosphate degradation